{
  "term_id": "GO:0008610",
  "term_label": "lipid biosynthetic process",
  "gene_name": "Alkyldihydroxyacetonephosphate synthase, peroxisomal",
  "gene": "UniProtKB:O00116",
  "gene_symbol": "AGPS"
}